muscle cell fate specification [GO:0042694] (biological process) Sources: CL:0000187, GOC:go_curators Definition: The process in which a cell becomes capable of differentiating autonomously into a muscle cell in an environment that is neutral with respect to the developmental pathway; upon specification, the cell fate can be reversed. Subtypes: vascular associated smooth muscle cell fate specification [GO:0097082] Relationships: is a type of GO:0001708; is part of muscle cell fate commitment [GO:0042693]